{
  "term_id": "GO:0030154",
  "gene_symbol": "PTK6",
  "term_label": "cell differentiation",
  "gene_name": "Protein-tyrosine kinase 6",
  "gene": "UniProtKB:Q13882"
}